{
  "term_label": "Unknown cellular component",
  "gene": "UniProtKB:Q9UK00",
  "term_id": "UNKNOWN:0003",
  "gene_symbol": "C3orf18",
  "gene_name": "Uncharacterized protein C3orf18"
}